{
  "term_id": "GO:0008076",
  "gene": "UniProtKB:Q03721",
  "gene_name": "Potassium voltage-gated channel subfamily C member 4",
  "term_label": "voltage-gated potassium channel complex",
  "gene_symbol": "KCNC4"
}